dUMP catabolic process [GO:0046079] (biological process) Also known as: dUMP breakdown, dUMP catabolism, dUMP degradation Relationships: is a type of pyrimidine deoxyribonucleoside monophosphate catabolic process [GO:0009178]; is a type of pyrimidine deoxyribonucleotide catabolic process [GO:0009223]; is a type of dUMP metabolic process [GO:0046078] Sources: GOC:go_curators Definition: The chemical reactions and pathways resulting in the breakdown of dUMP, deoxyuridine (5'-)monophosphate.